lateral loop [GO:0043219] (CC) Definition: Non-compact myelin located adjacent to the nodes of Ranvier in a myelin segment. These non-compact regions include cytoplasm from the cell responsible for synthesizing the myelin. Lateral loops are found in the paranodal region adjacent to the nodes of Ranvier, while Schmidt-Lantermann clefts are analogous structures found within the compact myelin internode. Sources: GOC:dgh Also known as: Schwann cell paranodal termination, oligodendrocyte paranodal termination, paranodal loop Relationships: is a type of GO:0110165; is part of myelin sheath [GO:0043209]